{
  "gene_name": "Ubiquitin-conjugating enzyme E2 K",
  "term_id": "GO:0000209",
  "term_label": "protein polyubiquitination",
  "gene_symbol": "UBE2K",
  "gene": "UniProtKB:P61086"
}